{
  "gene": "UniProtKB:Q96A72",
  "term_id": "GO:0008380",
  "term_label": "RNA splicing",
  "gene_name": "Protein mago nashi homolog 2",
  "gene_symbol": "MAGOHB"
}